{
  "term_id": "GO:0007411",
  "gene": "UniProtKB:O75326",
  "gene_name": "Semaphorin-7A",
  "gene_symbol": "SEMA7A",
  "term_label": "axon guidance"
}